{
  "gene_symbol": "CD44",
  "term_label": "hyaluronic acid binding",
  "gene_name": "CD44 antigen",
  "gene": "UniProtKB:P16070",
  "term_id": "GO:0005540"
}